{
  "gene_name": "43 kDa receptor-associated protein of the synapse",
  "gene_symbol": "RAPSN",
  "term_id": "GO:0007271",
  "gene": "UniProtKB:Q13702",
  "term_label": "synaptic transmission, cholinergic"
}